interferon-epsilon production [GO:0072647] (biological process) Note: Note that this term is in the subset of terms that should not be used for direct gene product annotation. Instead, select one of the 'regulation' children terms. References: PMID:15546383 Sources: GOC:BHF, GOC:mah Also known as: IFN-epsilon production, IFNE production, interferon-epsilon secretion Relationships: is a type of GO:0032606 Definition: The appearance of interferon-epsilon due to biosynthesis or secretion following a cellular stimulus, resulting in an increase in its intracellular or extracellular levels.